regulation of antifungal innate immune response [GO:1905034] (biological process) Subtypes: negative regulation of antifungal innate immune response [GO:1905035], positive regulation of antifungal innate immune response [GO:1905036] References: PMID:22470487 Sources: GOC:TermGenie, GOC:dph, GO_REF:0000058 Definition: Any process that modulates the frequency, rate or extent of an antifungal innate immune response. Relationships: is a type of regulation of innate immune response [GO:0045088]; is a type of regulation of defense response to fungus [GO:1900150]; regulates antifungal innate immune response [GO:0061760]